ABC-type manganese transporter activity [GO:0015410] (molecular function) Definition: Enables the transfer of a solute or solutes from one side of a membrane to the other according to the reaction: ATP + H2O + Mn2+(out) = ADP + phosphate + Mn2+(in). Sources: RHEA:17365 Also known as: ATP-dependent manganese transmembrane transporter activity, manganese ABC transporter, ABC-type Mn(2+) transporter, ATPase-coupled manganese transmembrane transporter activity, manganese transmembrane transporter activity, phosphorylative mechanism, manganese-transporting ATPase activity Relationships: is a type of manganese ion transmembrane transporter activity [GO:0005384]; is a type of ATPase-coupled monoatomic cation transmembrane transporter activity [GO:0019829]; is a type of GO:0140359